mononuclear cell differentiation [GO:1903131] (biological process) Relationships: is a type of leukocyte differentiation [GO:0002521] Definition: The process in which a relatively unspecialized cell acquires the specialized features of a mononuclear cell. References: PMID:24759906 Sources: CL:0000842, GOC:TermGenie, GO_REF:0000086 Subtypes: lymphocyte differentiation [GO:0030098], monocyte differentiation [GO:0030224], macrophage differentiation [GO:0030225], dendritic cell differentiation [GO:0097028]